{
  "term_id": "GO:0031593",
  "gene_name": "Ubiquilin-4",
  "gene_symbol": "UBQLN4",
  "term_label": "polyubiquitin modification-dependent protein binding",
  "gene": "UniProtKB:Q9NRR5"
}